sulfinoalanine decarboxylase activity [GO:0004782] (molecular function) Also known as: sulphinoalanine decarboxylase activity, 3-sulfino-L-alanine carboxy-lyase (hypotaurine-forming), 3-sulfino-L-alanine carboxy-lyase activity, CADCase/CSADCase activity, CSAD, CSADCase activity, L-cysteinesulfinic acid decarboxylase activity, cysteic decarboxylase activity, cysteine-sulfinate decarboxylase activity, cysteinesulfinate decarboxylase activity, cysteinesulfinic acid decarboxylase activity, sulfoalanine decarboxylase activity Relationships: is a type of carboxy-lyase activity [GO:0016831] Sources: EC:4.1.1.29 Definition: Catalysis of the reaction: 3-sulfino-L-alanine = hypotaurine + CO2.